transcytosis [GO:0045056] (biological process) Regulation: regulated by regulation of transcytosis [GO:1904298]; negatively regulated by GO:1904299; positively regulated by positive regulation of transcytosis [GO:1904300] Sources: ISBN:0716731363 Relationships: is a type of GO:0016192; is a type of multicellular organismal process [GO:0032501] Definition: The directed movement of endocytosed material through the cell and its exocytosis from the plasma membrane at the opposite side. Subtypes: antigen transcytosis by M cells in mucosal-associated lymphoid tissue [GO:0002412], immunoglobulin transcytosis in epithelial cells [GO:0002414], amyloid-beta clearance by transcytosis [GO:0150093]